{
  "term_id": "GO:0005886",
  "gene_symbol": "ALPL",
  "gene": "UniProtKB:P05186",
  "term_label": "plasma membrane",
  "gene_name": "Alkaline phosphatase, tissue-nonspecific isozyme"
}